{
  "term_id": "UNKNOWN:0002",
  "gene_symbol": "REELD1",
  "gene": "UniProtKB:A0A1B0GV85",
  "term_label": "Unknown biological process",
  "gene_name": "Reelin domain-containing protein 1"
}